{
  "term_label": "RNA polymerase II preinitiation complex assembly",
  "gene_symbol": "TAF1",
  "gene_name": "Transcription initiation factor TFIID subunit 1",
  "gene": "UniProtKB:P21675",
  "term_id": "GO:0051123"
}